{
  "term_label": "mediator complex",
  "gene": "UniProtKB:Q9Y2X0",
  "term_id": "GO:0016592",
  "gene_symbol": "MED16",
  "gene_name": "Mediator of RNA polymerase II transcription subunit 16"
}